{
  "gene_name": "Hemicentin-1",
  "term_id": "GO:0007157",
  "gene_symbol": "HMCN1",
  "gene": "UniProtKB:Q96RW7",
  "term_label": "heterophilic cell-cell adhesion"
}